{
  "gene_symbol": "TTLL8",
  "term_label": "spermatogenesis",
  "gene_name": "Protein monoglycylase TTLL8",
  "gene": "UniProtKB:A6PVC2",
  "term_id": "GO:0007283"
}